regulation of protein deubiquitination [GO:0090085] (biological process) Subtypes: GO:0090086, positive regulation of protein deubiquitination [GO:1903003], regulation of protein K63-linked deubiquitination [GO:1903004], GO:1903093 Relationships: is a type of regulation of protein modification by small protein conjugation or removal [GO:1903320]; regulates protein deubiquitination [GO:0016579] Definition: Any process that modulates the frequency, rate or extent of protein deubiquitination. Protein deubiquitination is the removal of one or more ubiquitin groups from a protein. Sources: GOC:BHF, GOC:dph, GOC:tb